sulfur amino acid transport [GO:0000101] (biological process) Also known as: sulphur amino acid transport Sources: GOC:ai Definition: The directed movement of amino acids containing sulfur (cystine, methionine and their derivatives) into, out of or within a cell, or between cells, by means of some agent such as a transporter or pore. Subtypes: L-cystine transport [GO:0015811], methionine transport [GO:0015821], cysteine transport [GO:0042883] Relationships: is_a carboxylic acid transport [GO:0046942]; is a type of nitrogen compound transport [GO:0071705]; is a type of sulfur compound transport [GO:0072348]